{
  "term_id": "UNKNOWN:0002",
  "term_label": "Unknown biological process",
  "gene_name": "Tigger transposable element-derived protein 3",
  "gene": "UniProtKB:Q6B0B8",
  "gene_symbol": "TIGD3"
}